{
  "gene_name": "Apolipoprotein A-IV",
  "term_id": "GO:0034362",
  "term_label": "low-density lipoprotein particle",
  "gene": "UniProtKB:P06727",
  "gene_symbol": "APOA4"
}